adenylyltransferase complex [GO:1902503] (CC) Subtypes: sulfate adenylyltransferase complex (ATP) [GO:0009336], GO:0010170, GO:1990133 References: PMID:11713534 Sources: GOC:TermGenie, GOC:bhm Also known as: ThiF-ThiS complex Definition: A protein complex which is capable of adenylyltransferase activity. Relationships: is a type of transferase complex, transferring phosphorus-containing groups [GO:0061695]